{
  "term_id": "GO:0005634",
  "gene_symbol": "PHF11",
  "term_label": "nucleus",
  "gene_name": "PHD finger protein 11",
  "gene": "UniProtKB:Q9UIL8"
}